chemokine (C-X-C motif) ligand 9 production [GO:0035393] (BP) Sources: GOC:add Also known as: CXCL9 production, MIG production, Monokine induced by gamma interferon production Relationships: is a type of chemokine production [GO:0032602] Definition: The appearance of chemokine (C-X-C motif) ligand 9 due to biosynthesis or secretion following a cellular stimulus, resulting in an increase in its intracellular or extracellular levels. Regulation: regulated by regulation of chemokine (C-X-C motif) ligand 9 production [GO:0035394]; RO_0002212 by negative regulation of chemokine (C-X-C motif) ligand 9 production [GO:0035395]; RO_0002213 by positive regulation of chemokine (C-X-C motif) ligand 9 production [GO:0035396]